{
  "gene_name": "KN motif and ankyrin repeat domain-containing protein 2",
  "gene_symbol": "KANK2",
  "gene": "UniProtKB:Q63ZY3",
  "term_label": "negative regulation of cell population proliferation",
  "term_id": "GO:0008285"
}